proximal tubule morphogenesis [GO:0072158] (biological process) Relationships: is a type of nephron tubule morphogenesis [GO:0072078]; is part of proximal tubule development [GO:0072014] Sources: GOC:mtg_kidney_jan10 Subtypes: pronephric proximal tubule morphogenesis [GO:0039011], mesonephric proximal tubule morphogenesis [GO:0061276], metanephric proximal tubule morphogenesis [GO:0072288] Definition: The process in which the anatomical structures of a proximal tubule are generated and organized. The proximal tubule is a nephron tubule that connects Bowman's capsule to the descending thin limb of the loop of Henle. It has a brush border epithelial morphology.